peptidoglycan-protein cross-linking [GO:0018104] (biological process) Definition: The process of covalently linking peptidoglycan (murein) to proteins. Sources: GOC:jsg Relationships: is a type of peptidoglycan biosynthetic process [GO:0009252]